{
  "gene": "UniProtKB:O95704",
  "gene_symbol": "APBB3",
  "term_id": "GO:0005737",
  "term_label": "cytoplasm",
  "gene_name": "Amyloid-beta A4 precursor protein-binding family B member 3"
}